{
  "gene_symbol": "DEFA3",
  "gene": "UniProtKB:P59666",
  "term_id": "GO:0005615",
  "gene_name": "Neutrophil defensin 3",
  "term_label": "extracellular space"
}